{
  "term_id": "UNKNOWN:0002",
  "gene": "UniProtKB:Q9Y5L5",
  "term_label": "Unknown biological process",
  "gene_name": "Lens epithelial cell protein LEP503",
  "gene_symbol": "LENEP"
}